{
  "gene_symbol": "TMEM262",
  "gene_name": "Cation channel sperm-associated auxiliary subunit TMEM262",
  "term_id": "UNKNOWN:0001",
  "term_label": "Unknown molecular function",
  "gene": "UniProtKB:E9PQX1"
}